supramolecular complex [GO:0099080] (cellular component) Subtypes: kinetochore [GO:0000776], aster [GO:0005818], ribonucleoprotein granule [GO:0035770], paraflagellar rod [GO:0097740], mastigoneme [GO:0097741], complex of collagen trimers [GO:0098644], supramolecular polymer [GO:0099081] Relationships: is a type of cellular anatomical structure [GO:0110165] Definition: A cellular component that consists of an indeterminate number of proteins or macromolecular complexes, organized into a regular, higher-order structure such as a polymer, sheet, network or a fiber. Sources: GOC:dos